{
  "term_label": "ISG15-protein conjugation",
  "term_id": "GO:0032020",
  "gene": "UniProtKB:Q9UII4",
  "gene_name": "E3 ISG15--protein ligase HERC5",
  "gene_symbol": "HERC5"
}